reductive iron assimilation [GO:0033215] (biological process) Definition: A process in which iron is solubilized by reduction from Fe3+ to Fe2+ via a cell surface reductase and subsequent transport of the iron across the membrane by iron uptake proteins. Also known as: iron assimilation by reduction and transport Relationships: is a type of GO:0033212; has part ferric-chelate reductase activity [GO:0000293]; has part iron ion transmembrane transport [GO:0034755] References: PMID:16963626 Sources: GOC:cjm, GOC:mah